{
  "gene": "UniProtKB:O43364",
  "term_label": "RNA polymerase II cis-regulatory region sequence-specific DNA binding",
  "gene_name": "Homeobox protein Hox-A2",
  "term_id": "GO:0000978",
  "gene_symbol": "HOXA2"
}